{
  "gene_symbol": "NMRK2",
  "gene_name": "Nicotinamide riboside kinase 2",
  "gene": "UniProtKB:Q9NPI5",
  "term_label": "ribosylnicotinamide kinase activity",
  "term_id": "GO:0050262"
}